viral DNA strand displacement replication [GO:0039687] (biological process) Sources: GOC:bf, GOC:jl, VZ:1940 Relationships: is a type of GO:0039693 Subtypes: rolling circle viral DNA replication [GO:0039682] Definition: A viral DNA replication process where only one strand is replicated at once, and which releases a single stranded DNA (ssDNA).